{
  "gene_symbol": "EEF1AKMT4-ECE2",
  "term_label": "metalloendopeptidase activity",
  "gene_name": "EEF1AKMT4-ECE2 readthrough transcript protein",
  "term_id": "GO:0004222",
  "gene": "UniProtKB:P0DPD8"
}